adrenergic receptor activity [GO:0004935] (molecular function) Sources: GOC:bf, GOC:mah, IUPHAR_GPCR:1274 Also known as: adrenoceptor activity Relationships: is a type of G protein-coupled amine receptor activity [GO:0008227]; is part of GO:0071875 Definition: Combining with epinephrine or norepinephrine and transmitting the signal across the membrane by activating the alpha-subunit of an associated heterotrimeric G-protein complex. Subtypes: alpha-adrenergic receptor activity [GO:0004936], beta-adrenergic receptor activity [GO:0004939]